L-arginine import across plasma membrane [GO:0097638] (biological process) Definition: The directed movement of L-arginine from outside of a cell, across the plasma membrane and into the cytosol. Regulation: regulated by GO:1905541; negatively regulated by negative regulation of L-arginine import across plasma membrane [GO:1905542]; positively regulated by positive regulation of L-arginine import across plasma membrane [GO:1905589] References: PMID:8195186 Sources: GOC:krc Also known as: arginine import, L-arginine import into cell Relationships: is a type of organic cation transport [GO:0015695]; is a type of amino acid import across plasma membrane [GO:0089718]; is a type of GO:1902475